{
  "gene": "UniProtKB:P55196",
  "term_label": "adherens junction",
  "term_id": "GO:0005912",
  "gene_symbol": "AFDN",
  "gene_name": "Afadin"
}